rRNA acetylation involved in maturation of SSU-rRNA [GO:1904812] (biological process) Relationships: is a type of rRNA acetylation [GO:1990882]; BFO_0000050 maturation of SSU-rRNA [GO:0030490] Definition: Any rRNA acetylation that is involved in maturation of SSU-rRNA. References: PMID:25402480 Sources: GOC:TermGenie, GO_REF:0000060 Also known as: rRNA acetylation involved in SSU-rRNA maturation, rRNA acetylation involved in processing of 20S pre-rRNA